{
  "gene_symbol": "ALKBH8",
  "term_label": "tRNA methylation",
  "term_id": "GO:0030488",
  "gene_name": "Alkylated DNA repair protein alkB homolog 8",
  "gene": "UniProtKB:Q96BT7"
}